{
  "gene_symbol": "SAGSIN1",
  "gene_name": "Salivary gland specific protein SAGSIN1",
  "term_label": "Unknown cellular component",
  "term_id": "UNKNOWN:0003",
  "gene": "UniProtKB:A0A0C4DGP1"
}